{
  "term_label": "RNA polymerase II cis-regulatory region sequence-specific DNA binding",
  "gene": "UniProtKB:Q96NI8",
  "gene_symbol": "ZNF570",
  "gene_name": "Zinc finger protein 570",
  "term_id": "GO:0000978"
}